{
  "term_id": "GO:0016020",
  "gene": "UniProtKB:Q9Y693",
  "gene_name": "LHFPL tetraspan subfamily member 6 protein",
  "term_label": "membrane",
  "gene_symbol": "LHFPL6"
}